embryo sac egg cell differentiation [GO:0009560] (biological process) Definition: The process in which an uncellularized embryo sac nucleus cellularizes and acquires the specialized features of an egg cell. An example of this process is found in Arabidopsis thaliana. Also known as: female gamete generation, female gametophyte egg cell differentiation Relationships: is_a developmental process involved in reproduction [GO:0003006]; is a type of cell differentiation [GO:0030154]; is part of female gamete generation [GO:0007292]; is part of megagametogenesis [GO:0009561] Regulation: regulated by GO:0045694; negatively regulated by GO:0045695; positively regulated by positive regulation of embryo sac egg cell differentiation [GO:0045696] Sources: GOC:jid, GOC:mtg_plant, GOC:mtg_sensu